lipopolysaccharide heptosyltransferase activity [GO:0008920] (molecular function) Relationships: is_a GO:0016757 Definition: Catalysis of the reaction: a lipopolysaccharide + ADP-L-glycero-beta-D-manno-heptose = a heptosylated lipopolysaccharide + ADP + H+. Subtypes: ADP-heptose-lipopolysaccharide heptosyltransferase activity [GO:0008713], GO:0071967, lipid A-core heptosyltransferase activity [GO:0071968] Also known as: LPS heptosyltransferase activity Sources: GOC:curators